4-toluenecarboxylate catabolic process [GO:0019612] (biological process) Relationships: is a type of benzene-containing compound metabolic process [GO:0042537]; is a type of monocarboxylic acid catabolic process [GO:0072329] Definition: The chemical reactions and pathways resulting in the breakdown of 4-toluenecarboxylate, 4-methylbenzenecarboxylate, the anion of carboxylic acid attached to a methylbenzene molecule. Also known as: 4-toluenecarboxylate breakdown, 4-toluenecarboxylate catabolism, 4-toluenecarboxylate degradation, p-toluate catabolic process, p-toluate catabolism Sources: GOC:ai